{
  "gene": "UniProtKB:Q6UX34",
  "gene_name": "Protein SNORC",
  "gene_symbol": "SNORC",
  "term_id": "UNKNOWN:0001",
  "term_label": "Unknown molecular function"
}